{
  "gene_symbol": "PCSK4",
  "gene_name": "Proprotein convertase subtilisin_kexin type 4",
  "term_label": "serine-type endopeptidase activity",
  "term_id": "GO:0004252",
  "gene": "UniProtKB:Q6UW60"
}